cell body membrane [GO:0044298] (cellular component) Sources: GOC:ecd Also known as: cell soma membrane Definition: The plasma membrane of a cell that bears surface projections such as axons, dendrites, cilia, or flagella, excluding the plasma membrane on cell projections. Subtypes: neuronal cell body membrane [GO:0032809] Relationships: is a type of cellular anatomical structure [GO:0110165]; is part of GO:0005886; is part of cell body [GO:0044297]